N-acylhexosamine oxidase activity [GO:0050122] (molecular function) Sources: EC:1.1.3.29, RHEA:13029 Relationships: is_a oxidoreductase activity, acting on the CH-OH group of donors, oxygen as acceptor [GO:0016899] Definition: Catalysis of the reaction: N-acetyl-D-glucosamine + H2O + O2 = N-acetyl-D-glucosaminate + H2O2 + H+. Also known as: N-acyl-D-hexosamine oxidase activity, N-acyl-D-hexosamine:oxygen 1-oxidoreductase activity, N-acyl-beta-D-hexosamine:oxygen 1-oxidoreductase activity